{
  "gene_name": "Cyclic AMP-responsive element-binding protein 3-like protein 1",
  "gene": "UniProtKB:Q96BA8",
  "gene_symbol": "CREB3L1",
  "term_label": "DNA-binding transcription factor activity, RNA polymerase II-specific",
  "term_id": "GO:0000981"
}